cellular response to mercury ion [GO:0071288] (biological process) Definition: Any process that results in a change in state or activity of a cell (in terms of movement, secretion, enzyme production, gene expression, etc.) as a result of a mercury ion stimulus. Relationships: is a type of response to mercury ion [GO:0046689]; is a type of GO:0071248 Also known as: cellular response to mercuric ion, cellular response to mercury Sources: GOC:mah